{
  "gene": "UniProtKB:O75155",
  "term_id": "GO:0016567",
  "gene_name": "Cullin-associated NEDD8-dissociated protein 2",
  "gene_symbol": "CAND2",
  "term_label": "protein ubiquitination"
}